{
  "gene": "UniProtKB:Q6IPM2",
  "gene_name": "IQ domain-containing protein E",
  "gene_symbol": "IQCE",
  "term_id": "UNKNOWN:0001",
  "term_label": "Unknown molecular function"
}